{
  "term_id": "GO:0005886",
  "term_label": "plasma membrane",
  "gene": "UniProtKB:O95977",
  "gene_name": "Sphingosine 1-phosphate receptor 4",
  "gene_symbol": "S1PR4"
}